{
  "term_id": "GO:0005737",
  "gene_name": "ADP-ribosylation factor-like protein 4D",
  "gene": "UniProtKB:P49703",
  "gene_symbol": "ARL4D",
  "term_label": "cytoplasm"
}